positive regulation of I-kappaB phosphorylation [GO:1903721] (biological process) Definition: Any process that activates or increases the frequency, rate or extent of I-kappaB phosphorylation. Also known as: positive regulation of IKB phosphorylation, positive regulation of IkappaB phosphorylation, positive regulation of inhibitor of NF-kappaB phosphorylation, positive regulation of inhibitor of kappaB phosphorylation, up regulation of I-kappaB phosphorylation, up regulation of IKB phosphorylation, up regulation of IkappaB phosphorylation, up regulation of inhibitor of NF-kappaB phosphorylation, up regulation of inhibitor of kappaB phosphorylation, up-regulation of I-kappaB phosphorylation, up-regulation of IKB phosphorylation, up-regulation of IkappaB phosphorylation, up-regulation of inhibitor of NF-kappaB phosphorylation, up-regulation of inhibitor of kappaB phosphorylation, upregulation of I-kappaB phosphorylation, upregulation of IKB phosphorylation, upregulation of IkappaB phosphorylation, upregulation of inhibitor of NF-kappaB phosphorylation, upregulation of inhibitor of kappaB phosphorylation, activation of I-kappaB phosphorylation, activation of IKB phosphorylation, activation of IkappaB phosphorylation, activation of inhibitor of NF-kappaB phosphorylation, activation of inhibitor of kappaB phosphorylation References: PMID:23675531 Sources: GOC:TermGenie, GO_REF:0000058 Relationships: is a type of positive regulation of protein phosphorylation [GO:0001934]; is a type of regulation of I-kappaB phosphorylation [GO:1903719]; positively regulates I-kappaB phosphorylation [GO:0007252]